{
  "term_label": "external side of plasma membrane",
  "term_id": "GO:0009897",
  "gene_name": "GDNF family receptor alpha-4",
  "gene": "UniProtKB:Q9GZZ7",
  "gene_symbol": "GFRA4"
}